coenzyme F420H2 oxidase activity [GO:0052765] (molecular function) Relationships: is a type of GO:0016647 Definition: Catalysis of the reaction: 2 reduced coenzyme F420-(gamma-L-Glu)(n) + O2 = 2 oxidized coenzyme F420-(gamma-L-Glu)(n) + 2 H2O + 2 H+. References: PMID:15340796 Sources: RHEA:39711 Also known as: F420H2 oxidase activity, F420H2:oxygen oxidoreductase activity, reduced coenzyme F420 oxidase activity